{
  "gene_symbol": "CUSTOS",
  "term_label": "Unknown cellular component",
  "gene_name": "Protein CUSTOS",
  "gene": "UniProtKB:Q96C57",
  "term_id": "UNKNOWN:0003"
}